{
  "term_id": "UNKNOWN:0001",
  "term_label": "Unknown molecular function",
  "gene_name": "Pinin",
  "gene_symbol": "PNN",
  "gene": "UniProtKB:Q9H307"
}